{
  "gene_name": "Calcium-responsive transcription factor",
  "gene_symbol": "CARF",
  "term_id": "GO:0000978",
  "term_label": "RNA polymerase II cis-regulatory region sequence-specific DNA binding",
  "gene": "UniProtKB:Q8N187"
}